phosphorelay signal transduction system [GO:0000160] (biological process) Relationships: is a type of intracellular signal transduction [GO:0035556] References: PMID:9191038 Regulation: regulated by GO:0070297; negatively regulated by negative regulation of phosphorelay signal transduction system [GO:0070298]; positively regulated by positive regulation of phosphorelay signal transduction system [GO:0070299] Definition: A conserved series of molecular signals found in prokaryotes and eukaryotes; involves autophosphorylation of a histidine kinase and the transfer of the phosphate group to an aspartate that then acts as a phospho-donor to response regulator proteins. Subtypes: osmosensory signaling via phosphorelay pathway [GO:0007234], ethylene-activated signaling pathway [GO:0009873] Also known as: histidyl-aspartyl phosphorelay